{
  "gene_name": "Microtubule-associated protein tau",
  "gene_symbol": "MAPT",
  "term_label": "neuron projection development",
  "gene": "UniProtKB:P10636",
  "term_id": "GO:0031175"
}